sesquiterpene biosynthetic process [GO:0051762] (biological process) Definition: The chemical reactions and pathways resulting in the formation of sesquiterpenes, any of a class of terpenes of the formula C15H24 or a derivative of such a terpene. Relationships: is a type of terpene biosynthetic process [GO:0046246]; is a type of sesquiterpene metabolic process [GO:0051761] Sources: GOC:ai Subtypes: culmorin biosynthetic process [GO:0106210], GO:1901928, alpha-copaene biosynthetic process [GO:1901931], bicyclogermacrene biosynthetic process [GO:1901934], beta-caryophyllene biosynthetic process [GO:1901937], (-)-exo-alpha-bergamotene biosynthetic process [GO:1901940]